{
  "gene_symbol": "CCZ1B",
  "term_id": "GO:0035658",
  "gene": "UniProtKB:P86790",
  "term_label": "Mon1-Ccz1 complex",
  "gene_name": "Vacuolar fusion protein CCZ1 homolog B"
}